{
  "term_id": "GO:0006376",
  "gene_symbol": "CELF2",
  "gene": "UniProtKB:O95319",
  "gene_name": "CUGBP Elav-like family member 2",
  "term_label": "mRNA splice site recognition"
}